{
  "gene_name": "E3 ubiquitin-protein ligase FANCL",
  "term_label": "protein monoubiquitination",
  "gene_symbol": "FANCL",
  "gene": "UniProtKB:Q9NW38",
  "term_id": "GO:0006513"
}